{
  "gene_symbol": "FH",
  "gene": "UniProtKB:P07954",
  "gene_name": "Fumarate hydratase, mitochondrial",
  "term_label": "tricarboxylic acid cycle",
  "term_id": "GO:0006099"
}